{
  "gene_symbol": "RFWD3",
  "term_label": "protein ubiquitination",
  "term_id": "GO:0016567",
  "gene_name": "E3 ubiquitin-protein ligase RFWD3",
  "gene": "UniProtKB:Q6PCD5"
}